{
  "gene": "UniProtKB:Q9UHQ7",
  "gene_name": "Transcription elongation factor A protein-like 9",
  "gene_symbol": "TCEAL9",
  "term_label": "Unknown cellular component",
  "term_id": "UNKNOWN:0003"
}